p53 binding [GO:0002039] (MF) Definition: Binding to one of the p53 family of proteins. Sources: GOC:hjd Relationships: is a type of protein binding [GO:0005515]